{
  "term_label": "Unknown cellular component",
  "gene": "UniProtKB:Q96EM0",
  "term_id": "UNKNOWN:0003",
  "gene_symbol": "L3HYPDH",
  "gene_name": "Trans-3-hydroxy-L-proline dehydratase"
}